{
  "term_label": "mitotic sister chromatid segregation",
  "gene": "UniProtKB:Q92674",
  "term_id": "GO:0000070",
  "gene_symbol": "CENPI",
  "gene_name": "Centromere protein I"
}